negative regulation of P-type sodium:potassium-exchanging transporter activity [GO:1903407] (biological process) Definition: Any process that stops, prevents or reduces the frequency, rate or extent of sodium:potassium-exchanging ATPase activity. References: PMID:8160880 Sources: GOC:TermGenie, GOC:mr, GO_REF:0000059 Also known as: down regulation of (Na+ + K+)-ATPase activity, down regulation of (Na+ + K+)-activated ATPase activity, down regulation of ATP phosphohydrolase (Na+/K+-exchanging), down regulation of Na(+)/K(+)-ATPase activity, down regulation of Na(+)/K(+)-exchanging ATPase activity, down regulation of Na+,K+-ATPase activity, down regulation of Na+/K+-ATPase activity, down regulation of Na+/K+-exchanging ATPase activity, down regulation of Na,K-activated ATPase activity, down regulation of sodium/potassium-exchanging ATPase activity, down regulation of sodium/potassium-transporting ATPase activity, down regulation of sodium:potassium exchanging ATPase activity, down regulation of sodium:potassium-exchanging ATPase activity, down-regulation of (Na+ + K+)-ATPase activity, down-regulation of (Na+ + K+)-activated ATPase activity, down-regulation of ATP phosphohydrolase (Na+/K+-exchanging), down-regulation of Na(+)/K(+)-ATPase activity, down-regulation of Na(+)/K(+)-exchanging ATPase activity, down-regulation of Na+,K+-ATPase activity, down-regulation of Na+/K+-ATPase activity, down-regulation of Na+/K+-exchanging ATPase activity, down-regulation of Na,K-activated ATPase activity, down-regulation of sodium/potassium-exchanging ATPase activity, down-regulation of sodium/potassium-transporting ATPase activity, down-regulation of sodium:potassium exchanging ATPase activity, down-regulation of sodium:potassium-exchanging ATPase activity, downregulation of (Na+ + K+)-ATPase activity, downregulation of (Na+ + K+)-activated ATPase activity, downregulation of ATP phosphohydrolase (Na+/K+-exchanging), downregulation of Na(+)/K(+)-ATPase activity, downregulation of Na(+)/K(+)-exchanging ATPase activity, downregulation of Na+,K+-ATPase activity, downregulation of Na+/K+-ATPase activity, downregulation of Na+/K+-exchanging ATPase activity, downregulation of Na,K-activated ATPase activity, downregulation of sodium/potassium-exchanging ATPase activity, downregulation of sodium/potassium-transporting ATPase activity, downregulation of sodium:potassium exchanging ATPase activity, downregulation of sodium:potassium-exchanging ATPase activity, negative regulation of (Na+ + K+)-ATPase activity, negative regulation of (Na+ + K+)-activated ATPase activity, negative regulation of ATP phosphohydrolase (Na+/K+-exchanging), negative regulation of Na(+)/K(+)-ATPase activity, negative regulation of Na(+)/K(+)-exchanging ATPase activity, negative regulation of Na+,K+-ATPase activity, negative regulation of Na+/K+-ATPase activity, negative regulation of Na+/K+-exchanging ATPase activity, negative regulation of Na,K-activated ATPase activity, negative regulation of sodium/potassium-exchanging ATPase activity, negative regulation of sodium/potassium-transporting ATPase activity, negative regulation of sodium:potassium exchanging ATPase activity, negative regulation of sodium:potassium-exchanging ATPase activity, inhibition of (Na+ + K+)-ATPase activity, inhibition of (Na+ + K+)-activated ATPase activity, inhibition of ATP phosphohydrolase (Na+/K+-exchanging), inhibition of Na(+)/K(+)-ATPase activity, inhibition of Na(+)/K(+)-exchanging ATPase activity, inhibition of Na+,K+-ATPase activity, inhibition of Na+/K+-ATPase activity, inhibition of Na+/K+-exchanging ATPase activity, inhibition of Na,K-activated ATPase activity, inhibition of sodium/potassium-exchanging ATPase activity, inhibition of sodium/potassium-transporting ATPase activity, inhibition of sodium:potassium exchanging ATPase activity, inhibition of sodium:potassium-exchanging ATPase activity, down regulation of Na+,K+ pump, down regulation of Na,K-pump, down-regulation of Na+,K+ pump, down-regulation of Na,K-pump, downregulation of Na+,K+ pump, downregulation of Na,K-pump, inhibition of Na+,K+ pump, inhibition of Na,K-pump, negative regulation of Na+,K+ pump, negative regulation of Na,K-pump Relationships: is_a negative regulation of ATP-dependent activity [GO:0032780]; is a type of negative regulation of potassium ion transmembrane transporter activity [GO:1901017]; is a type of regulation of P-type sodium:potassium-exchanging transporter activity [GO:1903406]; RO_0002212 GO:0005391